{
  "gene_symbol": "VTI1B",
  "gene": "UniProtKB:Q9UEU0",
  "term_id": "GO:0048280",
  "gene_name": "Vesicle transport through interaction with t-SNAREs homolog 1B",
  "term_label": "vesicle fusion with Golgi apparatus"
}